SCF-Met30/Pof1 ubiquitin ligase complex [GO:0097666] (cellular component) Relationships: is a type of SCF ubiquitin ligase complex [GO:0019005] References: PMID:15147268, PMID:9499404 Sources: GOC:jd, GOC:vw Definition: An SCF ubiquitin ligase complex in which the F-box protein is Met30 in S. cerevisiae (Pof1 in S pombe).